SRF-myogenin-E12 complex [GO:0070514] (cellular component) Relationships: is a type of RNA polymerase II transcription regulator complex [GO:0090575] Definition: A transcription factor complex that contains the serum response factor (SRF) and the basic helix-loop-helix proteins myogenin and E12, and is involved in activating transcription of muscle-specific genes. References: PMID:8617811